embryo sac morphogenesis [GO:0048314] (biological process) Relationships: is a type of GO:0048598; is part of megagametogenesis [GO:0009561] Definition: The process in which the anatomical structures of the embryo sac are generated and organized. The embryo sac develops from the megaspore in heterosporous plants. References: PMID:12271029, PMID:25332875 Sources: GOC:jid, GOC:mtg_plant Also known as: female gametophyte morphogenesis